lipophagy [GO:0061724] (biological process) Regulation: regulated by regulation of lipophagy [GO:1904502]; negatively regulated by GO:1904503; positively regulated by GO:1904504 Definition: The selective degradation of lipid droplets by macroautophagy. Relationships: is a type of macroautophagy [GO:0016236]; has part lipid droplet disassembly [GO:1905691] References: PMID:23708524, PMID:26076903 Sources: GOC:autophagy